{
  "gene_symbol": "CT45A1",
  "term_label": "Unknown cellular component",
  "term_id": "UNKNOWN:0003",
  "gene": "UniProtKB:Q5HYN5",
  "gene_name": "Cancer_testis antigen family 45 member A1"
}